{
  "gene": "UniProtKB:P31371",
  "gene_name": "Fibroblast growth factor 9",
  "term_id": "GO:0008284",
  "gene_symbol": "FGF9",
  "term_label": "positive regulation of cell population proliferation"
}